{
  "gene_symbol": "CXXC4",
  "term_label": "nucleus",
  "gene": "UniProtKB:Q9H2H0",
  "term_id": "GO:0005634",
  "gene_name": "CXXC-type zinc finger protein 4"
}